cytoplasmic exosome (RNase complex) [GO:0000177] (cellular component) Subtypes: bacterial degradosome [GO:1990061] Definition: A ribonuclease complex that has 3-prime to 5-prime processive hydrolytic exoribonuclease activity producing 5-prime-phosphomonoesters. Participates in a multitude of cellular RNA processing and degradation events preventing nuclear export and/or translation of aberrant RNAs. Restricted to processing linear and circular single-stranded RNAs (ssRNA) only. RNAs with complex secondary structures may have to be unwound or pre-processed by co-factors prior to entering the complex, esp if the 3-prime end is structured. Relationships: is_a GO:0000178; is part of cytoplasm [GO:0005737] References: PMID:17174896, PMID:20531386, PMID:26726035 Also known as: cytoplasmic exosome (ribonuclease complex), cytoplasmic exosome multienzyme ribonuclease complex, prokaryotic exosome multienzyme ribonuclease complex